nuclear pore organization [GO:0006999] (biological process) Definition: A process that is carried out at the cellular level which results in the assembly, arrangement of constituent parts, or disassembly of the nuclear pore. Relationships: is a type of nucleus organization [GO:0006997]; is a type of protein-containing complex organization [GO:0043933] Also known as: nuclear pore organisation, nuclear pore complex organization and biogenesis, nuclear pore organization and biogenesis Sources: GOC:dph, GOC:jid, GOC:jl, GOC:mah Subtypes: GO:0051292, mitotic nuclear pore complex disassembly [GO:0140516]